{
  "term_id": "GO:1902358",
  "gene_name": "Solute carrier family 26 member 6",
  "gene": "UniProtKB:Q9BXS9",
  "term_label": "sulfate transmembrane transport",
  "gene_symbol": "SLC26A6"
}